detoxification of cadmium ion [GO:0071585] (biological process) Definition: Any process that reduces or removes the toxicity of cadmium ion. These may include transport of cadmium away from sensitive areas and to compartments or complexes whose purpose is sequestration of cadmium ion. Relationships: is a type of detoxification of inorganic compound [GO:0061687]; is part of stress response to cadmium ion [GO:1990170] Subtypes: cellular detoxification of cadmium ion [GO:0098849] References: PMID:16741752 Sources: GOC:BHF, GOC:kmv